{
  "term_id": "GO:0008209",
  "gene_name": "3-hydroxyacyl-CoA dehydrogenase type-2",
  "term_label": "androgen metabolic process",
  "gene": "UniProtKB:Q99714",
  "gene_symbol": "HSD17B10"
}